{
  "term_id": "GO:0003682",
  "gene_symbol": "ACTRT1",
  "gene": "UniProtKB:Q8TDG2",
  "gene_name": "Actin-related protein T1",
  "term_label": "chromatin binding"
}